thiamine diphosphate dephosphorylation [GO:0042370] (biological process) Definition: The removal of one or more phosphate groups from thiamine diphosphate, a derivative of thiamine (vitamin B1) which acts as a coenzyme in a range of processes including the Krebs cycle. Sources: GOC:jl, ISBN:0198506732 Also known as: TPP dephosphorylation, thiamin diphosphate dephosphorylation Relationships: is a type of thiamine diphosphate metabolic process [GO:0042357]